guanine deaminase activity [GO:0008892] (molecular function) Relationships: is a type of hydrolase activity, acting on carbon-nitrogen (but not peptide) bonds, in cyclic amidines [GO:0016814]; is_a deaminase activity [GO:0019239] Also known as: GAH activity, guanase activity, guanine aminase activity, guanine aminohydrolase activity Sources: EC:3.5.4.3 Definition: Catalysis of the reaction: guanine + H2O = xanthine + NH3.